{
  "term_label": "mitochondrial transcription factor activity",
  "gene_name": "Dimethyladenosine transferase 1, mitochondrial",
  "gene_symbol": "TFB1M",
  "term_id": "GO:0034246",
  "gene": "UniProtKB:Q8WVM0"
}